{
  "term_id": "GO:0000978",
  "gene_name": "Nuclear factor 1 C-type",
  "term_label": "RNA polymerase II cis-regulatory region sequence-specific DNA binding",
  "gene_symbol": "NFIC",
  "gene": "UniProtKB:P08651"
}